{
  "term_label": "mitochondrial outer membrane",
  "gene": "UniProtKB:Q8TB36",
  "gene_name": "Ganglioside-induced differentiation-associated protein 1",
  "gene_symbol": "GDAP1",
  "term_id": "GO:0005741"
}